homologous chromosome segregation [GO:0045143] (biological process) Regulation: RO_0002211 by regulation of homologous chromosome segregation [GO:0060629] Relationships: is a type of meiotic chromosome segregation [GO:0045132]; BFO_0000050 meiosis I [GO:0007127] Sources: GOC:ai, ISBN:0815316194 Definition: The cell cycle process in which replicated homologous chromosomes are organized and then physically separated and apportioned to two sets during the first division of the meiotic cell cycle. Each replicated chromosome, composed of two sister chromatids, aligns at the cell equator, paired with its homologous partner; this pairing off, referred to as synapsis, permits genetic recombination. One homolog (both sister chromatids) of each morphologic type goes into each of the resulting chromosome sets. Also known as: meiosis I, chromosome segregation